{
  "gene_name": "Unconventional myosin-XV",
  "gene_symbol": "MYO15A",
  "term_label": "microfilament motor activity",
  "gene": "UniProtKB:Q9UKN7",
  "term_id": "GO:0000146"
}